CCA tRNA nucleotidyltransferase activity [GO:0004810] (MF) Definition: Catalysis of the reaction: a tRNA precursor + ATP + 2 CTP = a tRNA with a 3' CCA end + 3 diphosphate. References: PMID:2247609 Sources: RHEA:14433 Also known as: ATP(CTP)-tRNA nucleotidyltransferase, ATP(CTP):tRNA nucleotidyltransferase activity, CTP(ATP):tRNA nucleotidyltransferase, CTP:tRNA cytidylyltransferase activity, ribonucleic cytidylic cytidylic adenylic pyrophosphorylase, ribonucleic cytidylyltransferase, tRNA adenylyl(cytidylyl)transferase, tRNA-nucleotidyltransferase activity, transfer RNA adenylyltransferase, transfer ribonucleate adenylyltransferase, transfer ribonucleate nucleotidyltransferase, transfer ribonucleic acid nucleotidyl transferase, transfer ribonucleic adenylyl (cytidylyl) transferase, transfer ribonucleic-terminal trinucleotide nucleotidyltransferase, transfer-RNA nucleotidyltransferase, CCA-adding enzyme activity, tRNA CCA-diphosphorylase activity, tRNA cytidylyltransferase activity, transfer ribonucleate adenyltransferase activity Relationships: is a type of GO:0070567; is a type of catalytic activity, acting on a tRNA [GO:0140101]